{
  "gene": "UniProtKB:Q9UI40",
  "gene_name": "Sodium_potassium_calcium exchanger 2",
  "term_label": "intracellular calcium ion homeostasis",
  "gene_symbol": "SLC24A2",
  "term_id": "GO:0006874"
}